{
  "term_label": "Unknown molecular function",
  "gene_symbol": "LRRC20",
  "gene": "UniProtKB:Q8TCA0",
  "term_id": "UNKNOWN:0001",
  "gene_name": "Leucine-rich repeat-containing protein 20"
}